{
  "gene_symbol": "NETO2",
  "gene": "UniProtKB:Q8NC67",
  "gene_name": "Neuropilin and tolloid-like protein 2",
  "term_id": "GO:0099645",
  "term_label": "neurotransmitter receptor localization to postsynaptic specialization membrane"
}